{
  "gene_name": "Dexamethasone-induced protein",
  "gene_symbol": "DEXI",
  "term_id": "UNKNOWN:0002",
  "term_label": "Unknown biological process",
  "gene": "UniProtKB:O95424"
}